{
  "term_label": "cytosol",
  "gene": "UniProtKB:P49591",
  "term_id": "GO:0005829",
  "gene_name": "Serine--tRNA ligase, cytoplasmic",
  "gene_symbol": "SARS1"
}